{
  "gene_name": "Neurite extension and migration factor",
  "gene_symbol": "NEXMIF",
  "term_id": "GO:0001953",
  "term_label": "negative regulation of cell-matrix adhesion",
  "gene": "UniProtKB:Q5QGS0"
}